{
  "gene": "UniProtKB:Q7L1T6",
  "gene_name": "Cytochrome b5 reductase 4",
  "term_label": "superoxide metabolic process",
  "term_id": "GO:0006801",
  "gene_symbol": "CYB5R4"
}